{
  "gene": "UniProtKB:O00418",
  "term_label": "regulation of translation at postsynapse",
  "gene_name": "Eukaryotic elongation factor 2 kinase",
  "gene_symbol": "EEF2K",
  "term_id": "GO:0140245"
}